{
  "gene_symbol": "SLITRK1",
  "term_label": "axonogenesis",
  "term_id": "GO:0007409",
  "gene": "UniProtKB:Q96PX8",
  "gene_name": "SLIT and NTRK-like protein 1"
}